{
  "gene": "UniProtKB:O43345",
  "term_label": "nucleus",
  "gene_symbol": "ZNF208",
  "gene_name": "Zinc finger protein 208",
  "term_id": "GO:0005634"
}